subtelomeric heterochromatin formation [GO:0031509] (biological process) Definition: The compaction of chromatin into heterochromatin at the subtelomeric region. References: PMID:10219245, PMID:26205977 Sources: GOC:mah Also known as: Telomere Position Effect, chromatin silencing at telomere, heterochromatic silencing at telomere, subtelomeric heterochromatin assembly, subtelomeric silencing, telomere chromatin silencing, telomeric silencing, chromatin silencing at subtelomere, establishment of chromatin silencing at telomere, heterochromatic silencing at subtelomere, regulation of chromatin silencing at telomere, regulation of subtelomeric heterochromatin assembly, subtelomere chromatin silencing, telomeric heterochromatin assembly, telomeric heterochromatin formation Relationships: is a type of constitutive heterochromatin formation [GO:0140719]; occurs in GO:0000781